{
  "term_label": "protein maturation",
  "gene_name": "NFU1 iron-sulfur cluster scaffold homolog, mitochondrial",
  "term_id": "GO:0051604",
  "gene_symbol": "NFU1",
  "gene": "UniProtKB:Q9UMS0"
}